{
  "gene_symbol": "SNU13",
  "term_id": "GO:0031428",
  "term_label": "box C/D methylation guide snoRNP complex",
  "gene_name": "NHP2-like protein 1",
  "gene": "UniProtKB:P55769"
}